endoplasmic reticulum to cytosol transport [GO:1903513] (biological process) Also known as: ER to cytosol transport References: PMID:16402920 Sources: GOC:BHF, GOC:TermGenie, GOC:mtg_cardiac_conduct_nov11, GOC:rl, GO_REF:0000076 Relationships: is a type of intracellular transport [GO:0046907] Subtypes: retrograde protein transport, ER to cytosol [GO:0030970] Definition: The directed movement of substances from endoplasmic reticulum to cytosol.